follicle cell of egg chamber-cell adhesion [GO:0007299] (biological process) References: PMID:12642496 Sources: GOC:bf, GOC:mtg_sensu Definition: The attachment of a somatic follicle cell to another somatic follicle cell or to its substratum, the germline cells. An example of this is found in Drosophila melanogaster. Also known as: follicle cell adhesion, ovarian follicle cell adhesion Relationships: is a type of GO:0090136; is part of follicle cell of egg chamber development [GO:0030707]